N-acetylglucosaminyldiphosphoundecaprenol N-acetyl-beta-D-mannosaminyltransferase activity [GO:0047244] (molecular function) Relationships: is a type of GO:0008194; is a type of hexosyltransferase activity [GO:0016758] Also known as: N-acetylmannosaminyltransferase activity, UDP-N-acetyl-D-mannosamine:N-acetyl-beta-D-glucosaminyldiphosphoundecaprenol beta-1,4-N-acetylmannosaminyltransferase activity, UDP-N-acetylmannosamine:N-acetylglucosaminyl diphosphorylundecaprenol N-acetylmannosaminyltransferase activity, uridine diphosphoacetyl-mannosamineacetylglucosaminylpyrophosphorylundecaprenol acetylmannosaminyltransferase activity Definition: Catalysis of the reaction: N-acetyl-D-glucosaminyldiphosphoundecaprenol + UDP-N-acetyl-D-mannosamine = N-acetyl-beta-D-mannosaminyl-1,4-N-acetyl-D-glucosaminyldiphosphoundecaprenol + UDP. Sources: EC:2.4.1.187